{
  "gene_name": "T cell receptor alpha joining 17 (Fragment)",
  "term_label": "Unknown molecular function",
  "gene": "UniProtKB:A0A075B6W8",
  "term_id": "UNKNOWN:0001",
  "gene_symbol": "TRAJ17"
}